{
  "gene_symbol": "KIF5C",
  "term_id": "GO:0005874",
  "gene_name": "Kinesin heavy chain isoform 5C",
  "gene": "UniProtKB:O60282",
  "term_label": "microtubule"
}